collagen type XII trimer [GO:0005595] (cellular component) References: PMID:21421911 Definition: A collagen homotrimer of alpha1(XII) chains; type XII collagen triple helices may link sheet-forming or fibrillar collagens to other structures. Relationships: is a type of FACIT collagen trimer [GO:0005593]